mitotic G1 DNA damage checkpoint signaling [GO:0031571] (biological process) Definition: A signal transduction process that contributes to a mitotic cell cycle G1/S transition DNA damage checkpoint. Relationships: is a type of GO:0044773; is a type of mitotic G1/S transition checkpoint signaling [GO:0044819]; happens during mitotic G1 phase [GO:0000080] Sources: GOC:mtg_cell_cycle Also known as: intracellular signal transduction involved in G1 DNA damage checkpoint, intracellular signal transduction involved in G1/S DNA damage checkpoint, intracellular signal transduction pathway involved in G1 DNA damage checkpoint, intracellular signal transduction pathway involved in G1/S DNA damage checkpoint, intracellular signaling cascade involved in G1 DNA damage checkpoint, intracellular signaling cascade involved in G1/S DNA damage checkpoint, intracellular signaling chain involved in G1 DNA damage checkpoint, intracellular signaling chain involved in G1/S DNA damage checkpoint, intracellular signaling pathway involved in G1 DNA damage checkpoint, intracellular signaling pathway involved in G1/S DNA damage checkpoint, mitotic G1 DNA damage checkpoint, mitotic cell cycle G1/S transition DNA damage checkpoint, signal transduction via intracellular signaling cascade involved in G1 DNA damage checkpoint, signal transduction via intracellular signaling cascade involved in G1/S DNA damage checkpoint, signal transmission via intracellular cascade involved in G1 DNA damage checkpoint, G1 DNA damage checkpoint, G1/S DNA damage checkpoint, signal transduction involved in mitotic G1 DNA damage checkpoint, signal transduction involved in mitotic cell cycle G1/S transition DNA damage checkpoint